{
  "gene_name": "POU domain, class 6, transcription factor 1",
  "term_id": "UNKNOWN:0003",
  "term_label": "Unknown cellular component",
  "gene": "UniProtKB:Q14863",
  "gene_symbol": "POU6F1"
}